{
  "gene_symbol": "KCTD1",
  "term_id": "GO:0005634",
  "gene": "UniProtKB:Q719H9",
  "gene_name": "BTB_POZ domain-containing protein KCTD1",
  "term_label": "nucleus"
}